{
  "gene": "UniProtKB:Q9C0D3",
  "gene_symbol": "ZYG11B",
  "term_id": "GO:0031462",
  "term_label": "Cul2-RING ubiquitin ligase complex",
  "gene_name": "Protein zyg-11 homolog B"
}